{
  "gene_name": "Cyclin-I2",
  "term_id": "GO:0000307",
  "term_label": "cyclin-dependent protein kinase holoenzyme complex",
  "gene_symbol": "CCNI2",
  "gene": "UniProtKB:Q6ZMN8"
}